{
  "gene": "UniProtKB:Q16819",
  "term_label": "metalloendopeptidase activity",
  "gene_symbol": "MEP1A",
  "gene_name": "Meprin A subunit alpha",
  "term_id": "GO:0004222"
}